{
  "gene_symbol": "OLFM2",
  "term_label": "Unknown molecular function",
  "gene_name": "Noelin-2",
  "term_id": "UNKNOWN:0001",
  "gene": "UniProtKB:O95897"
}